{
  "gene": "UniProtKB:Q8NGC2",
  "gene_symbol": "OR4E2",
  "gene_name": "Olfactory receptor 4E2",
  "term_label": "olfactory receptor activity",
  "term_id": "GO:0004984"
}